bursa of Fabricius development [GO:0048540] (biological process) Definition: The process whose specific outcome is the progression of the bursa of Fabricius over time, from its formation to the mature structure. The bursa of Fabricius is an organ found in birds involved in B cell differentiation. Sources: GOC:add, ISBN:0781735149 Relationships: is a type of hematopoietic or lymphoid organ development [GO:0048534]